{
  "gene_name": "Testis-specific Y-encoded protein 10",
  "gene_symbol": "TSPY10",
  "term_label": "nucleus",
  "gene": "UniProtKB:P0CW01",
  "term_id": "GO:0005634"
}